{
  "gene_name": "Palladin",
  "gene_symbol": "PALLD",
  "gene": "UniProtKB:Q8WX93",
  "term_label": "cell-cell adhesion mediator activity",
  "term_id": "GO:0098632"
}